{
  "gene": "UniProtKB:Q5W111",
  "term_id": "UNKNOWN:0001",
  "gene_name": "SPRY domain-containing protein 7",
  "term_label": "Unknown molecular function",
  "gene_symbol": "SPRYD7"
}